{
  "gene_name": "High affinity cAMP-specific 3',5'-cyclic phosphodiesterase 7A",
  "term_label": "Unknown cellular component",
  "gene": "UniProtKB:Q13946",
  "gene_symbol": "PDE7A",
  "term_id": "UNKNOWN:0003"
}